renal outer medulla development [GO:0072054] (biological process) Also known as: outer renal medulla development Sources: GOC:mtg_kidney_jan10 Relationships: is_a anatomical structure development [GO:0048856]; BFO_0000050 kidney development [GO:0001822] Definition: The process whose specific outcome is the progression of the renal outer medulla over time, from its formation to the mature structure. The renal outer medulla is the region of the kidney that lies between the renal cortex and the renal inner medulla.